{
  "term_label": "SNARE binding",
  "gene_name": "Protein transport protein Sec24D",
  "gene": "UniProtKB:O94855",
  "term_id": "GO:0000149",
  "gene_symbol": "SEC24D"
}